{
  "gene_name": "26S proteasome non-ATPase regulatory subunit 11",
  "gene_symbol": "PSMD11",
  "gene": "UniProtKB:O00231",
  "term_id": "GO:0006511",
  "term_label": "ubiquitin-dependent protein catabolic process"
}